{
  "term_id": "UNKNOWN:0002",
  "gene_name": "CYFIP-related Rac1 interactor A",
  "gene": "UniProtKB:Q9H0Q0",
  "term_label": "Unknown biological process",
  "gene_symbol": "CYRIA"
}